high-affinity sodium:dicarboxylate symporter activity [GO:0015362] (molecular function) Relationships: is a type of GO:0017153 Also known as: high affinity sodium:dicarboxylate cotransporter activity, high affinity sodium:dicarboxylate symporter activity Definition: Enables the transfer of a solute or solutes from one side of a membrane to the other according to the reaction: dicarboxylate(out) + Na+(out) = dicarboxylate(in) + Na+(in). In high-affinity transport the transporter is able to bind the solute even if it is only present at very low concentrations. Sources: TC:2.A.47.1.4